{
  "term_id": "GO:0005886",
  "term_label": "plasma membrane",
  "gene_symbol": "CD59",
  "gene": "UniProtKB:P13987",
  "gene_name": "CD59 glycoprotein"
}